{
  "gene_name": "DnaJ homolog subfamily B member 7",
  "gene": "UniProtKB:Q7Z6W7",
  "gene_symbol": "DNAJB7",
  "term_label": "protein folding",
  "term_id": "GO:0006457"
}